{
  "gene": "UniProtKB:Q03052",
  "term_id": "UNKNOWN:0003",
  "gene_name": "POU domain, class 3, transcription factor 1",
  "gene_symbol": "POU3F1",
  "term_label": "Unknown cellular component"
}